hexadecanal metabolic process [GO:0046458] (biological process) Definition: The chemical reactions and pathways involving hexadecanal, the C16 straight chain aldehyde. References: PMID:25047030 Also known as: hexadecanal metabolism Relationships: is a type of aldehyde metabolic process [GO:0006081] Subtypes: GO:0006634